{
  "gene_symbol": "ITGBL1",
  "gene": "UniProtKB:O95965",
  "term_label": "cell surface",
  "gene_name": "Integrin beta-like protein 1",
  "term_id": "GO:0009986"
}